{
  "gene_symbol": "RAB8B",
  "gene_name": "Ras-related protein Rab-8B",
  "gene": "UniProtKB:Q92930",
  "term_label": "exocytosis",
  "term_id": "GO:0006887"
}